{
  "gene": "UniProtKB:Q9BRJ9",
  "gene_name": "Mesoderm posterior protein 1",
  "gene_symbol": "MESP1",
  "term_id": "GO:0006357",
  "term_label": "regulation of transcription by RNA polymerase II"
}